{
  "term_label": "cytosol",
  "term_id": "GO:0005829",
  "gene_name": "Ubiquitin carboxyl-terminal hydrolase 29",
  "gene": "UniProtKB:Q9HBJ7",
  "gene_symbol": "USP29"
}